anterior cell cortex [GO:0061802] (cellular component) Definition: The region that lies just beneath the plasma membrane in the part of a cell that is closest to the anterior as defined by the developing, or existing, anterior/posterior axis. Relationships: is a type of cell cortex region [GO:0099738] Sources: GOC:15666355, GOC:17981131, GOC:dph, GOC:kmv